paracrine signaling [GO:0038001] (biological process) Sources: GOC:mtg_signaling_feb11, ISBN:3527303782 Note: This term should be used with caution, and only used when the signaling between cells has been clearly distinguished from endocrine signaling. Also known as: paracrine signalling Relationships: is_a cell-cell signaling [GO:0007267] Definition: The transfer of information from one cell to another, where the signal travels from the signal-producing cell to the receiving cell by passive diffusion or bulk flow in intercellular fluid. The signaling cell and the receiving cell are usually in the vicinity of each other.